{
  "term_id": "GO:0004438",
  "gene": "UniProtKB:Q9NYA4",
  "gene_name": "Myotubularin-related protein 4",
  "gene_symbol": "MTMR4",
  "term_label": "phosphatidylinositol-3-phosphate phosphatase activity"
}